{
  "gene_name": "High affinity cGMP-specific 3',5'-cyclic phosphodiesterase 9A",
  "term_id": "UNKNOWN:0003",
  "term_label": "Unknown cellular component",
  "gene_symbol": "PDE9A",
  "gene": "UniProtKB:O76083"
}